{
  "gene_name": "Immunoglobulin kappa variable 1-17",
  "term_label": "immune response",
  "term_id": "GO:0006955",
  "gene_symbol": "IGKV1-17",
  "gene": "UniProtKB:P01599"
}